copper ion export from vacuole [GO:0140145] (biological process) References: PMID:12244050 Sources: GOC:vw Relationships: is a type of vacuolar transmembrane transport [GO:0034486]; is a type of copper ion transmembrane transport [GO:0035434] Definition: The directed movement of copper ions out of the vacuole across the vacuolar membrane.